meiotic sister chromatid cohesion, centromeric [GO:0051754] (biological process) Also known as: centromeric meiotic sister chromatin cohesion, meiotic sister chromatid cohesion at centromere, sister chromatid cohesion at centromere at meiosis I Relationships: is a type of GO:0051177; is a type of centromeric sister chromatid cohesion [GO:0070601] References: PMID:14730319, PMID:16325576 Definition: The cell cycle process in which centromeres of sister chromatids are joined during meiosis.